{
  "gene": "UniProtKB:P55769",
  "gene_symbol": "SNU13",
  "term_label": "U4/U6 x U5 tri-snRNP complex",
  "gene_name": "NHP2-like protein 1",
  "term_id": "GO:0046540"
}